{
  "gene": "UniProtKB:Q9C0I3",
  "gene_symbol": "CCSER1",
  "gene_name": "Serine-rich coiled-coil domain-containing protein 1",
  "term_id": "UNKNOWN:0002",
  "term_label": "Unknown biological process"
}